estrone sulfotransferase activity [GO:0004304] (molecular function) Definition: Catalysis of the reaction: 3'-phosphoadenosine 5'-phosphosulfate + estrone = adenosine 3',5'-bisphosphate + estrone 3-sulfate. Sources: EC:2.8.2.4 Also known as: estrogen sulfotransferase, estrone sulphotransferase activity, 3'-phosphoadenylyl sulfate-estrone 3-sulfotransferase activity, 3'-phosphoadenylyl-sulfate:estrone 3-sulfotransferase activity, 3'-phosphoadenylylsulfate:oestrone sulfotransferase activity, estrogen sulphotransferase activity, oestrogen sulphotransferase activity Relationships: is a type of sulfotransferase activity [GO:0008146]